{
  "gene": "UniProtKB:Q9BXC9",
  "term_id": "GO:0043005",
  "term_label": "neuron projection",
  "gene_symbol": "BBS2",
  "gene_name": "Bardet-Biedl syndrome 2 protein"
}